{
  "term_label": "lymph vessel development",
  "gene_name": "Transmembrane protein 204",
  "term_id": "GO:0001945",
  "gene": "UniProtKB:Q9BSN7",
  "gene_symbol": "TMEM204"
}